{
  "term_label": "ESCRT II complex",
  "gene_name": "Vacuolar protein-sorting-associated protein 36",
  "gene_symbol": "VPS36",
  "gene": "UniProtKB:Q86VN1",
  "term_id": "GO:0000814"
}